{
  "gene_symbol": "AQP2",
  "gene_name": "Aquaporin-2",
  "gene": "UniProtKB:P41181",
  "term_label": "water channel activity",
  "term_id": "GO:0015250"
}